metanephric early distal convoluted tubule development [GO:0072222] (biological process) Relationships: is a type of early distal convoluted tubule development [GO:0072067]; is a type of metanephric nephron epithelium development [GO:0072243]; is part of metanephric distal convoluted tubule development [GO:0072221] Definition: The process whose specific outcome is the progression of the metanephric early distal convoluted tubule over time, from its formation to the mature structure. The metanephric early distal convoluted tubule contains metanephric DCT cells and is vasopressin-insensitive. Sources: GOC:mtg_kidney_jan10